{
  "term_label": "actin filament binding",
  "gene": "UniProtKB:Q8IVF7",
  "gene_symbol": "FMNL3",
  "term_id": "GO:0051015",
  "gene_name": "Formin-like protein 3"
}